{
  "gene_symbol": "SMG9",
  "gene_name": "Nonsense-mediated mRNA decay factor SMG9",
  "gene": "UniProtKB:Q9H0W8",
  "term_id": "GO:0000184",
  "term_label": "nuclear-transcribed mRNA catabolic process, nonsense-mediated decay"
}